{
  "gene_name": "Ubiquitin-like modifier-activating enzyme 1",
  "gene": "UniProtKB:P22314",
  "term_id": "GO:0004839",
  "gene_symbol": "UBA1",
  "term_label": "ubiquitin activating enzyme activity"
}